cellular response to stress [GO:0033554] (biological process) Sources: GOC:mah Subtypes: DNA damage response [GO:0006974], GO:0009267, GO:0009626, negative regulation of ribosomal protein gene transcription from RNA polymerase II promoter in response to stress [GO:0010690], stress-activated protein kinase signaling cascade [GO:0031098], neuron projection regeneration [GO:0031102], GO:0034605, response to endoplasmic reticulum stress [GO:0034976], cellular response to isolation stress [GO:0035901], cellular response to immobilization stress [GO:0035903], cellular response to topologically incorrect protein [GO:0035967], cellular response to cell envelope stress [GO:0036460], DNA protection [GO:0042262], cellular response to water deprivation [GO:0042631], GO:0052482, cellular response to caloric restriction [GO:0061433], cellular response to chemical stress [GO:0062197], GO:0070417, cellular response to anoxia [GO:0071454], cellular response to hypoxia [GO:0071456], cellular response to fluid shear stress [GO:0071498], cellular response to sterol depletion [GO:0071501], response to mitochondrial depolarisation [GO:0098780], stress-induced homeostatically regulated protein degradation pathway [GO:0120174], cellular response to actin cytoskeletal stress [GO:0120306], integrated stress response signaling [GO:0140467], GO:0160144, stress-induced mitochondrial fusion [GO:1990046] Relationships: is a type of response to stress [GO:0006950]; is a type of cellular response to stimulus [GO:0051716] Regulation: regulated by regulation of cellular response to stress [GO:0080135] Definition: Any process that results in a change in state or activity of a cell (in terms of movement, secretion, enzyme production, gene expression, etc.) as a result of a stimulus indicating the organism is under stress. The stress is usually, but not necessarily, exogenous (e.g. temperature, humidity, ionizing radiation).